{
  "term_id": "GO:0016324",
  "gene_name": "ATP-binding cassette sub-family G member 5",
  "term_label": "apical plasma membrane",
  "gene": "UniProtKB:Q9H222",
  "gene_symbol": "ABCG5"
}